{
  "term_id": "GO:0017148",
  "gene_name": "Polyadenylate-binding protein-interacting protein 2",
  "term_label": "negative regulation of translation",
  "gene_symbol": "PAIP2",
  "gene": "UniProtKB:Q9BPZ3"
}